positive regulation of cell wall polysaccharide catabolic process [GO:2000968] (biological process) Sources: GOC:mengo_curators Subtypes: positive regulation of plant-type cell wall cellulose catabolic process [GO:2000941], positive regulation of mannan catabolic process [GO:2000996] Definition: Any process that activates or increases the frequency, rate or extent of cell wall polysaccharide catabolic process. Also known as: positive regulation of cell wall polysaccharide breakdown Relationships: is a type of positive regulation of catabolic process [GO:0009896]; is a type of GO:0010604; is a type of GO:0045913; is_a regulation of cell wall polysaccharide catabolic process [GO:2000966]; positively regulates cell wall polysaccharide catabolic process [GO:0044347]